{
  "gene": "UniProtKB:O15054",
  "term_label": "histone H3K27me2/H3K27me3 demethylase activity",
  "gene_symbol": "KDM6B",
  "gene_name": "Lysine-specific demethylase 6B",
  "term_id": "GO:0071558"
}